{
  "gene": "UniProtKB:P57087",
  "gene_name": "Junctional adhesion molecule B",
  "gene_symbol": "JAM2",
  "term_id": "GO:0005886",
  "term_label": "plasma membrane"
}